{
  "gene_name": "Cytochrome P450 1A2",
  "term_label": "xenobiotic catabolic process",
  "gene_symbol": "CYP1A2",
  "term_id": "GO:0042178",
  "gene": "UniProtKB:P05177"
}